glutaminyl-tRNA synthase (glutamine-hydrolyzing) activity [GO:0050567] (molecular function) Relationships: is a type of GO:0016884; is_a GO:0140101 Definition: Catalysis of the reaction: L-glutamine + glutamyl-tRNA(Gln) + ATP = L-glutamate + glutaminyl-tRNA(Gln) + phosphate + ADP. Sources: EC:6.3.5.7, MetaCyc:6.3.5.7-RXN Also known as: Glu-AdT activity, Glu-tRNA(Gln) amidotransferase activity, Glu-tRNAGln amidotransferase activity, Glu-tRNAGln:L-glutamine amido-ligase (ADP-forming), glutaminyl-tRNA synthase (glutamine-hydrolysing), glutamyl-tRNA(Gln) amidotransferase activity, glutamyl-tRNAGln amidotransferase activity, glutamyl-tRNAGln:L-glutamine amido-ligase (ADP-forming)